beta-catenin binding [GO:0008013] (molecular function) Relationships: is a type of GO:0005515 Sources: GOC:bf Definition: Binding to a catenin beta subunit.